epistomal sclerite development [GO:0048724] (BP) Definition: The process whose specific outcome is the progression of the epistomal sclerite over time, from its formation to the mature structure. Sources: GOC:rc Relationships: is a type of GO:0048856; is part of clypeo-labral disc development [GO:0035213]